{
  "gene_symbol": "LYPD2",
  "gene_name": "Ly6_PLAUR domain-containing protein 2",
  "term_label": "Unknown biological process",
  "term_id": "UNKNOWN:0002",
  "gene": "UniProtKB:Q6UXB3"
}